{
  "gene_name": "Gamma-crystallin B",
  "gene_symbol": "CRYGB",
  "gene": "UniProtKB:P07316",
  "term_label": "visual perception",
  "term_id": "GO:0007601"
}